{
  "gene_symbol": "CELSR2",
  "gene_name": "Cadherin EGF LAG seven-pass G-type receptor 2",
  "term_label": "adherens junction",
  "gene": "UniProtKB:Q9HCU4",
  "term_id": "GO:0005912"
}